{
  "gene": "UniProtKB:Q969M1",
  "term_label": "mitochondrial outer membrane translocase complex",
  "gene_name": "Mitochondrial import receptor subunit TOM40B",
  "gene_symbol": "TOMM40L",
  "term_id": "GO:0005742"
}